lipid digestion [GO:0044241] (biological process) Definition: The whole of the physical, chemical, and biochemical processes carried out by living organisms to break down ingested lipids into components that may be easily absorbed and directed into metabolism. Sources: GOC:go_curators Relationships: is a type of digestion [GO:0007586]